{
  "gene_symbol": "FOXC1",
  "gene_name": "Forkhead box protein C1",
  "gene": "UniProtKB:Q12948",
  "term_id": "GO:0006357",
  "term_label": "regulation of transcription by RNA polymerase II"
}